{
  "term_label": "ciliary basal body",
  "gene_name": "Protein BCAP",
  "gene": "UniProtKB:Q9ULJ1",
  "term_id": "GO:0036064",
  "gene_symbol": "ODF2L"
}